{
  "term_label": "chemical synaptic transmission",
  "gene_name": "5-hydroxytryptamine receptor 1A",
  "gene_symbol": "HTR1A",
  "term_id": "GO:0007268",
  "gene": "UniProtKB:P08908"
}